response to fenofibrate [GO:1901557] (biological process) Definition: Any process that results in a change in state or activity of a cell or an organism (in terms of movement, secretion, enzyme production, gene expression, etc.) as a result of a fenofibrate stimulus. Sources: GOC:TermGenie Relationships: is a type of response to ether [GO:0045472]; is a type of response to ketone [GO:1901654]